neuronal dense core vesicle exocytosis [GO:0099011] (biological process) Subtypes: presynaptic dense core vesicle exocytosis [GO:0099525], GO:0150038 References: PMID:17553987, PMID:24653208 Sources: GOC:kmv Relationships: is_a dense core granule exocytosis [GO:1990504] Definition: The secretion of molecules (e.g. neuropeptides, insulin-related peptides or neuromodulators such as serotonin and dopamine) contained within a neuronal dense core vesicle by fusion of the granule with the plasma membrane of a neuron in response to increased cytosolic calcium levels.